T cell receptor complex [GO:0042101] (cellular component) Definition: A protein complex that contains a disulfide-linked heterodimer of T cell receptor (TCR) chains, which are members of the immunoglobulin superfamily, and mediates antigen recognition, ultimately resulting in T cell activation. The TCR heterodimer is associated with the CD3 complex, which consists of the nonpolymorphic polypeptides gamma, delta, epsilon, zeta, and, in some cases, eta (an RNA splice variant of zeta) or Fc epsilon chains. Sources: GOC:mah, ISBN:0781735149 Also known as: T lymphocyte receptor complex, T-cell receptor complex, T-lymphocyte receptor complex, TCR complex, TCR Relationships: is a type of plasma membrane signaling receptor complex [GO:0098802] Subtypes: GO:0042105, gamma-delta T cell receptor complex [GO:0042106]